N-acetylglucosamine-6-phosphate deacetylase activity [GO:0008448] (molecular function) Definition: Catalysis of the reaction: H2O + N-acetyl-D-glucosamine 6-phosphate = acetate + D-glucosamine 6-phosphate. Sources: RHEA:22936 Also known as: 2-acetamido-2-deoxy-D-glucose-6-phosphate amidohydrolase activity, N-acetyl-D-glucosamine-6-phosphate amidohydrolase activity, acetylaminodeoxyglucosephosphate acetylhydrolase activity, acetylglucosamine phosphate deacetylase activity Relationships: is a type of hydrolase activity, acting on carbon-nitrogen (but not peptide) bonds, in linear amides [GO:0016811]; is a type of deacetylase activity [GO:0019213]